{
  "term_label": "Unknown molecular function",
  "gene_symbol": "FAM166A",
  "term_id": "UNKNOWN:0001",
  "gene": "UniProtKB:Q6J272",
  "gene_name": "Protein FAM166A"
}